{
  "term_label": "Unknown biological process",
  "gene": "UniProtKB:Q7Z2Y8",
  "gene_symbol": "GVINP1",
  "gene_name": "Interferon-induced very large GTPase 1",
  "term_id": "UNKNOWN:0002"
}